{
  "term_label": "translation initiation factor activity",
  "gene_symbol": "EIF3B",
  "gene_name": "Eukaryotic translation initiation factor 3 subunit B",
  "term_id": "GO:0003743",
  "gene": "UniProtKB:P55884"
}